positive regulation of protein-glutamine gamma-glutamyltransferase activity [GO:0150074] (biological process) Relationships: is a type of positive regulation of catalytic activity [GO:0043085]; is_a regulation of transferase activity [GO:0051338]; positively regulates protein-glutamine gamma-glutamyltransferase activity [GO:0003810] References: PMID:26670206 Sources: GOC:aruk, GOC:bc Definition: Any process that activates or increases the frequency, rate or extent of protein-glutamine gamma-glutamyltransferase activity.